{
  "gene_symbol": "GSTM2",
  "term_id": "GO:0004364",
  "gene": "UniProtKB:P28161",
  "term_label": "glutathione transferase activity",
  "gene_name": "Glutathione S-transferase Mu 2"
}